{
  "term_id": "GO:0005886",
  "term_label": "plasma membrane",
  "gene": "UniProtKB:C9JDP6",
  "gene_symbol": "CLDN25",
  "gene_name": "Putative claudin-25"
}